{
  "gene_symbol": "CENPVL3",
  "gene_name": "Centromere protein V-like protein 3",
  "term_id": "UNKNOWN:0003",
  "gene": "UniProtKB:A0A0U1RRI6",
  "term_label": "Unknown cellular component"
}